{
  "term_id": "GO:0000122",
  "gene_name": "Protein HEXIM2",
  "gene_symbol": "HEXIM2",
  "term_label": "negative regulation of transcription by RNA polymerase II",
  "gene": "UniProtKB:Q96MH2"
}